{
  "term_id": "GO:0048306",
  "gene_name": "Protein S100-A13",
  "term_label": "calcium-dependent protein binding",
  "gene": "UniProtKB:Q99584",
  "gene_symbol": "S100A13"
}